{
  "term_id": "UNKNOWN:0002",
  "term_label": "Unknown biological process",
  "gene_symbol": "FAM171B",
  "gene": "UniProtKB:Q6P995",
  "gene_name": "Protein FAM171B"
}